prosthetic group metabolic process [GO:0051189] (biological process) Subtypes: molybdopterin cofactor metabolic process [GO:0043545], GO:0051190, prosthetic group biosynthetic process [GO:0051191] Sources: GOC:ai Also known as: coenzyme and prosthetic group metabolic process, coenzyme and prosthetic group metabolism, prosthetic group metabolism Relationships: is a type of GO:0008152; BFO_0000050 protein metabolic process [GO:0019538] Definition: The chemical reactions and pathways involving a prosthetic group, the non-amino acid portion of certain protein molecules. Prosthetic groups may be inorganic or organic and are usually required for the biological activity of the protein.